{
  "gene_name": "Protein KHNYN",
  "term_label": "RNA endonuclease activity",
  "gene": "UniProtKB:O15037",
  "gene_symbol": "KHNYN",
  "term_id": "GO:0004521"
}